hippurate hydrolase activity [GO:0047980] (molecular function) Sources: EC:3.5.1.32, RHEA:10424 Relationships: is a type of hydrolase activity, acting on carbon-nitrogen (but not peptide) bonds, in linear amides [GO:0016811] Also known as: N-benzoylamino-acid amidohydrolase activity, benzoylglycine amidohydrolase activity, hippuricase activity Definition: Catalysis of the reaction: N-benzoylglycine + H2O = benzoate + glycine.